{
  "gene": "UniProtKB:Q9BX59",
  "term_id": "GO:0023024",
  "term_label": "MHC class I protein complex binding",
  "gene_symbol": "TAPBPL",
  "gene_name": "Tapasin-related protein"
}